{
  "gene": "UniProtKB:O43716",
  "term_label": "Unknown molecular function",
  "gene_name": "Glutamyl-tRNA(Gln) amidotransferase subunit C, mitochondrial",
  "term_id": "UNKNOWN:0001",
  "gene_symbol": "GATC"
}